capsanthin biosynthetic process [GO:1901809] (biological process) Definition: The chemical reactions and pathways resulting in the formation of capsanthin. References: PMID:10995282 Sources: GOC:TermGenie, GOC:yaf, MetaCyc:PWY-5174, UniPathway:UPA00806 Also known as: capsanthin anabolism, capsanthin biosynthesis, capsanthin formation, capsanthin synthesis Relationships: is a type of xanthophyll biosynthetic process [GO:0016123]